{
  "gene": "UniProtKB:A0A1B0GTB2",
  "term_label": "Unknown molecular function",
  "gene_symbol": "TUNAR",
  "term_id": "UNKNOWN:0001",
  "gene_name": "Protein TUNAR"
}